positive regulation of interferon-alpha production [GO:0032727] (biological process) Also known as: up regulation of interferon-alpha production, up-regulation of interferon-alpha production, upregulation of interferon-alpha production, activation of interferon-alpha production, positive regulation of interferon-alpha biosynthetic process, positive regulation of interferon-alpha secretion, stimulation of interferon-alpha production References: PMID:15546383 Sources: GOC:mah Relationships: is a type of GO:0032481; is a type of GO:0032647; positively regulates interferon-alpha production [GO:0032607] Definition: Any process that activates or increases the frequency, rate, or extent of interferon-alpha production.